{
  "gene_name": "Guanine nucleotide-binding protein G(t) subunit alpha-1",
  "gene_symbol": "GNAT1",
  "term_id": "GO:0001664",
  "term_label": "G protein-coupled receptor binding",
  "gene": "UniProtKB:P11488"
}